{
  "term_label": "sensory perception of sound",
  "term_id": "GO:0007605",
  "gene_name": "Glutaredoxin domain-containing cysteine-rich protein 2",
  "gene_symbol": "GRXCR2",
  "gene": "UniProtKB:A6NFK2"
}